{
  "term_id": "UNKNOWN:0002",
  "gene": "UniProtKB:Q68D86",
  "gene_name": "Coiled-coil domain-containing protein 102B",
  "term_label": "Unknown biological process",
  "gene_symbol": "CCDC102B"
}